RISC-loading complex [GO:0070578] (cellular component) References: PMID:18178619, PMID:19820710 Sources: GOC:BHF, GOC:ab, GOC:nc, GOC:rph Relationships: is a type of endoribonuclease complex [GO:1902555] Also known as: miRLC, microRNA loading complex, RLC Definition: A trimeric protein complex required for the formation of a mature RNA-induced silencing complex (RISC). In humans the complex is composed of the endonuclease Dicer (DICER1), TRBP (TARBP2) and the Argonaute protein Ago2 (EIF2C2/AGO2). Within the complex, Dicer and TRBP are required to process precursor miRNAs (pre-miRNAs) to mature miRNAs and then load them onto Ago2. Ago2 bound to the mature miRNA constitutes the minimal RISC and may subsequently dissociate from Dicer and TRBP. This complex has endoribonuclease activity.